{
  "gene_name": "Forkhead box protein F2",
  "term_label": "RNA polymerase II cis-regulatory region sequence-specific DNA binding",
  "term_id": "GO:0000978",
  "gene_symbol": "FOXF2",
  "gene": "UniProtKB:Q12947"
}